bioactive lipid receptor activity [GO:0045125] (molecular function) Subtypes: GO:0038036, lysophosphatidic acid receptor activity [GO:0070915] Definition: Combining with a bioactive lipid and transmitting the signal across the membrane by activating an associated G-protein; promotes the exchange of GDP for GTP on the alpha subunit of a heterotrimeric G-protein complex. A bioactive lipid is a lipid for which changes in lipid levels result in functional consequences in a variety of cellular processes. Relationships: is a type of G protein-coupled receptor activity [GO:0004930] References: PMID:12215548, PMID:18216770 Sources: GOC:bf, GOC:mah